{
  "term_label": "Unknown cellular component",
  "gene_name": "Interleukin-1 receptor-associated kinase 1-binding protein 1",
  "gene_symbol": "IRAK1BP1",
  "term_id": "UNKNOWN:0003",
  "gene": "UniProtKB:Q5VVH5"
}